{
  "gene_name": "Adenosine receptor A1",
  "term_label": "dendrite",
  "gene": "UniProtKB:P30542",
  "gene_symbol": "ADORA1",
  "term_id": "GO:0030425"
}